flavin reductase (NADH) activity [GO:0036382] (molecular function) Relationships: is a type of oxidoreductase activity, acting on the CH-NH group of donors, NAD or NADP as acceptor [GO:0016646] Sources: GOC:rs, RHEA:31303 Definition: Catalysis of the reaction: a reduced flavin + NAD+ = an oxidized flavin + 2 H+ + NADH.